trans-4-hexen-3-one reductase activity [GO:0102236] (molecular function) References: PMID:21169366 Sources: GOC:pz Definition: Catalysis of the reaction: trans-4-hexen-3-one + NADPH + H+ = hexan-3-one + NADP. Relationships: is a type of GO:0016628